{
  "gene_name": "CCA tRNA nucleotidyltransferase 1, mitochondrial",
  "term_id": "GO:0001680",
  "gene": "UniProtKB:Q96Q11",
  "term_label": "tRNA 3'-terminal CCA addition",
  "gene_symbol": "TRNT1"
}